oxoacid metabolic process [GO:0043436] (biological process) Definition: The chemical reactions and pathways involving any oxoacid; an oxoacid is a compound which contains oxygen, at least one other element, and at least one hydrogen bound to oxygen, and which produces a conjugate base by loss of positive hydrogen ion(s) (hydrons). Relationships: is a type of organic acid metabolic process [GO:0006082] Also known as: keto acid metabolic process, keto acid metabolism, ketoacid metabolic process, ketoacid metabolism, oxo acid metabolic process, oxo acid metabolism, oxoacid metabolism Sources: Wikipedia:Oxyacid Subtypes: hypochlorous acid biosynthetic process [GO:0002149], hypochlorous acid catabolic process [GO:0002150], polyphosphate metabolic process [GO:0006797], GO:0018892, dodecyl sulfate metabolic process [GO:0018909], glyphosate metabolic process [GO:0018920], organic phosphonate metabolic process [GO:0019634], carboxylic acid metabolic process [GO:0019752], glucosinolate metabolic process [GO:0019760], nitrate metabolic process [GO:0042126], 3'-phosphoadenosine 5'-phosphosulfate metabolic process [GO:0050427], diphosphate metabolic process [GO:0071344]